{
  "gene_symbol": "RTN4",
  "gene_name": "Reticulon-4",
  "term_id": "GO:0043005",
  "term_label": "neuron projection",
  "gene": "UniProtKB:Q9NQC3"
}